meiotic strand invasion involved in reciprocal meiotic recombination [GO:0010774] (biological process) Sources: GOC:dph, GOC:tb Definition: The cell cycle process in which double strand breaks are formed and repaired through a double Holliday junction intermediate resulting in meiotic recombination. Meiotic recombination is the cell cycle process in which double strand breaks are formed and repaired through a double Holliday junction intermediate. Relationships: is a type of meiotic strand invasion [GO:0000708]; BFO_0000050 reciprocal meiotic recombination [GO:0007131]